{
  "gene_name": "Heart- and neural crest derivatives-expressed protein 1",
  "term_label": "RNA polymerase II transcription regulatory region sequence-specific DNA binding",
  "gene_symbol": "HAND1",
  "gene": "UniProtKB:O96004",
  "term_id": "GO:0000977"
}